{
  "gene_symbol": "ANKRD52",
  "gene": "UniProtKB:Q8NB46",
  "term_label": "Unknown molecular function",
  "gene_name": "Serine_threonine-protein phosphatase 6 regulatory ankyrin repeat subunit C",
  "term_id": "UNKNOWN:0001"
}